smooth endoplasmic reticulum [GO:0005790] (cellular component) Sources: ISBN:0198506732 Relationships: is a type of GO:0005783 Also known as: SER, smooth ER Definition: The smooth endoplasmic reticulum (smooth ER or SER) has no ribosomes attached to it. The smooth ER is the recipient of the proteins synthesized in the rough ER. Those proteins to be exported are passed to the Golgi complex, the resident proteins are returned to the rough ER and the lysosomal proteins after phosphorylation of their mannose residues are passed to the lysosomes. Glycosylation of the glycoproteins also continues. The smooth ER is the site of synthesis of lipids, including the phospholipids. The membranes of the smooth ER also contain enzymes that catalyze a series of reactions to detoxify both lipid-soluble drugs and harmful products of metabolism. Large quantities of certain compounds such as phenobarbital cause an increase in the amount of the smooth ER.